{
  "gene_symbol": "PAX5",
  "gene": "UniProtKB:Q02548",
  "term_id": "GO:0000978",
  "term_label": "RNA polymerase II cis-regulatory region sequence-specific DNA binding",
  "gene_name": "Paired box protein Pax-5"
}